positive regulation of vascular associated smooth muscle cell migration [GO:1904754] (biological process) References: PMID:20693317 Sources: GOC:BHF, GOC:BHF_miRNA, GOC:TermGenie, GOC:rph, GO_REF:0000058 Also known as: positive regulation of vascular smooth muscle cell migration, up regulation of vascular associated smooth muscle cell migration, up regulation of vascular smooth muscle cell migration, up-regulation of vascular associated smooth muscle cell migration, up-regulation of vascular smooth muscle cell migration, upregulation of vascular associated smooth muscle cell migration, upregulation of vascular smooth muscle cell migration, activation of vascular associated smooth muscle cell migration, activation of vascular smooth muscle cell migration Relationships: is a type of positive regulation of smooth muscle cell migration [GO:0014911]; is a type of regulation of vascular associated smooth muscle cell migration [GO:1904752]; positively regulates vascular associated smooth muscle cell migration [GO:1904738] Definition: Any process that activates or increases the frequency, rate or extent of vascular associated smooth muscle cell migration.